sorocarp stalk cell differentiation [GO:0031149] (biological process) Also known as: stalk cell differentiation Definition: The process in which a relatively unspecialized cell acquires specialized features of a sorocarp stalk cell, any of the cellulose-covered cells that form the stalk of a sorocarp. An example of this process is found in Dictyostelium discoideum. References: PMID:4338436 Sources: GOC:mah, GOC:mtg_sensu, ISBN:0521583640 Relationships: is a type of cell differentiation [GO:0030154]; is part of sorocarp stalk development [GO:0031150] Regulation: regulated by regulation of sorocarp stalk cell differentiation [GO:0031285]; negatively regulated by negative regulation of sorocarp stalk cell differentiation [GO:0031286]; RO_0002213 by positive regulation of sorocarp stalk cell differentiation [GO:0031287]